{
  "gene_symbol": "TRAV22",
  "gene_name": "T cell receptor alpha variable 22",
  "gene": "UniProtKB:A0A0B4J277",
  "term_label": "Unknown biological process",
  "term_id": "UNKNOWN:0002"
}